{
  "term_label": "centrosome",
  "gene": "UniProtKB:Q8N4C6",
  "gene_symbol": "NIN",
  "gene_name": "Ninein",
  "term_id": "GO:0005813"
}